{
  "gene_name": "Ras-associating and dilute domain-containing protein",
  "gene": "UniProtKB:Q96JH8",
  "term_id": "GO:0001755",
  "gene_symbol": "RADIL",
  "term_label": "neural crest cell migration"
}